{
  "gene_name": "Nuclear factor 1 X-type",
  "term_id": "GO:0000981",
  "term_label": "DNA-binding transcription factor activity, RNA polymerase II-specific",
  "gene_symbol": "NFIX",
  "gene": "UniProtKB:Q14938"
}